{
  "gene_symbol": "PTGR1",
  "term_id": "UNKNOWN:0003",
  "term_label": "Unknown cellular component",
  "gene": "UniProtKB:Q14914",
  "gene_name": "Prostaglandin reductase 1"
}